{
  "gene": "UniProtKB:O75077",
  "term_id": "GO:0042734",
  "gene_symbol": "ADAM23",
  "term_label": "presynaptic membrane",
  "gene_name": "Disintegrin and metalloproteinase domain-containing protein 23"
}